adamantanone catabolic process [GO:0019263] (biological process) Sources: GOC:ai Definition: The chemical reactions and pathways resulting in the breakdown of adamantanone, tricyclo(3.3.1.13,7)decanone, a white crystalline solid used as an intermediate for microelectronics in the production of photoresists. Relationships: is a type of xenobiotic catabolic process [GO:0042178]; is a type of ketone catabolic process [GO:0042182] Also known as: adamantanone breakdown, adamantanone catabolism, adamantanone degradation